regulation of foraging behavior [GO:1903368] (biological process) Relationships: is a type of regulation of behavior [GO:0050795]; RO_0002211 GO:0060756 References: PMID:8677262 Sources: GOC:TermGenie, GOC:mr, GO_REF:0000058 Subtypes: negative regulation of foraging behavior [GO:1903369], positive regulation of foraging behavior [GO:1903370] Definition: Any process that modulates the frequency, rate or extent of foraging behavior.